{
  "gene_symbol": "CDC14A",
  "term_id": "GO:0004725",
  "gene": "UniProtKB:Q9UNH5",
  "gene_name": "Dual specificity protein phosphatase CDC14A",
  "term_label": "protein tyrosine phosphatase activity"
}